host cell cytoplasm part [GO:0033655] (cellular component) Definition: Any constituent part of the host cell cytoplasm, all of the contents of a cell excluding the plasma membrane and nucleus, but including other subcellular structures. The host is defined as the larger of the organisms involved in a symbiotic interaction. Sources: GOC:pamgo_curators Also known as: cytoplasm component Note: Note that this term is in the subset of terms that should not be used for direct gene product annotation. Instead, select a child term or, if no appropriate child term exists, please request a new term. Direct annotations to this term may be amended during annotation QC. Relationships: is_a host intracellular part [GO:0033646]; is part of host cell cytoplasm [GO:0030430] Subtypes: GO:0020030, Maurer's cleft [GO:0020036], host cell mitochondrion [GO:0033650], cytoplasmic viral factory [GO:0039714], host symbiosome [GO:0043658], host thylakoid membrane [GO:0044160], GO:0044161, host cell cytoplasmic vesicle membrane [GO:0044162], host cell cytosol [GO:0044164], host cell endoplasmic reticulum [GO:0044165], host cell endoplasmic reticulum lumen [GO:0044166], GO:0044172, host cell endosome [GO:0044174], GO:0044177, GO:0044186, GO:0044187, host cell mitochondrial envelope [GO:0044190], GO:0044220, double membrane vesicle viral factory lumen [GO:0062244], GO:0072492, GO:0072493, tubovesicular membrane network [GO:0085026], GO:0120149